{
  "gene_symbol": "SELE",
  "term_label": "heterophilic cell-cell adhesion",
  "gene_name": "E-selectin",
  "term_id": "GO:0007157",
  "gene": "UniProtKB:P16581"
}